{
  "term_label": "catenin complex",
  "gene": "UniProtKB:Q9HBT6",
  "gene_name": "Cadherin-20",
  "term_id": "GO:0016342",
  "gene_symbol": "CDH20"
}